thalianol metabolic process [GO:0080003] (biological process) References: PMID:18356490 Definition: The chemical reactions and pathways involving the triterpene thalianol. Relationships: is_a triterpenoid metabolic process [GO:0006722] Also known as: thalianol metabolism